{
  "gene_symbol": "PFDN5",
  "gene": "UniProtKB:Q99471",
  "term_id": "GO:1990113",
  "gene_name": "Prefoldin subunit 5",
  "term_label": "RNA polymerase I assembly"
}